{
  "gene": "UniProtKB:A6NFY7",
  "gene_name": "Succinate dehydrogenase assembly factor 1, mitochondrial",
  "term_id": "UNKNOWN:0001",
  "gene_symbol": "SDHAF1",
  "term_label": "Unknown molecular function"
}